{
  "gene_symbol": "DCST1",
  "term_id": "UNKNOWN:0003",
  "gene_name": "E3 ubiquitin-protein ligase DCST1",
  "term_label": "Unknown cellular component",
  "gene": "UniProtKB:Q5T197"
}